anterior cibarial plate morphogenesis [GO:0048717] (biological process) Sources: GOC:rc Relationships: is a type of post-embryonic animal morphogenesis [GO:0009886]; is part of clypeo-labral disc morphogenesis [GO:0007453]; is part of anterior cibarial plate development [GO:0048722] Definition: The process in which the anatomical structures of the anterior cibarial plate are generated and organized.